vitamin D3 biosynthetic process [GO:1901755] (biological process) Sources: GOC:TermGenie, GOC:yaf, Unipathway:UPA00955 Definition: The chemical reactions and pathways resulting in the formation of vitamin D3. Also known as: calciol anabolism, calciol biosynthesis, calciol biosynthetic process, calciol formation, calciol synthesis, cholecalciferol biosynthesis, cholecalciferol biosynthetic process, vitamin D3 anabolism, vitamin D3 biosynthesis, vitamin D3 formation, vitamin D3 synthesis Relationships: is_a GO:0042368; is a type of vitamin D3 metabolic process [GO:0070640]; is a type of GO:0120178; is a type of secondary alcohol biosynthetic process [GO:1902653]